{
  "gene_symbol": "RBM20",
  "gene": "UniProtKB:Q5T481",
  "term_id": "GO:0003729",
  "term_label": "mRNA binding",
  "gene_name": "RNA-binding protein 20"
}